{
  "term_label": "microtubule",
  "gene_symbol": "KIF3C",
  "gene_name": "Kinesin-like protein KIF3C",
  "term_id": "GO:0005874",
  "gene": "UniProtKB:O14782"
}